{
  "gene": "UniProtKB:Q8N1D0",
  "term_id": "UNKNOWN:0001",
  "term_label": "Unknown molecular function",
  "gene_symbol": "SLC22A18AS",
  "gene_name": "Beckwith-Wiedemann syndrome chromosomal region 1 candidate gene B protein"
}